eosinophil activation involved in immune response [GO:0002278] (biological process) Sources: GOC:add, ISBN:0781735149 Definition: The change in morphology and behavior of a eosinophil resulting from exposure to a cytokine, chemokine, cellular ligand, or soluble factor, leading to the initiation or perpetuation of an immune response. Also known as: eosinophil activation during immune response Relationships: is a type of myeloid cell activation involved in immune response [GO:0002275]; is a type of eosinophil activation [GO:0043307]